{
  "term_label": "Unknown biological process",
  "gene_name": "Cystatin-M",
  "gene_symbol": "CST6",
  "gene": "UniProtKB:Q15828",
  "term_id": "UNKNOWN:0002"
}